methyl fluoride metabolic process [GO:0018929] (biological process) Definition: The chemical reactions and pathways involving methyl fluoride, fluorine-substituted methane, a gaseous halogenated hydrocarbon that has been investigated as an inhibitor of methanotrophy and nitrification in soils. Sources: UM-BBD_pathwayID:mf Relationships: is a type of halogenated hydrocarbon metabolic process [GO:0042197]; is a type of organofluorine metabolic process [GO:0090346] Also known as: methyl fluoride metabolism